{
  "gene_symbol": "PATE4",
  "term_label": "Unknown biological process",
  "gene": "UniProtKB:P0C8F1",
  "gene_name": "Prostate and testis expressed protein 4",
  "term_id": "UNKNOWN:0002"
}